{
  "gene_name": "Rho-related GTP-binding protein RhoC",
  "term_id": "GO:0005829",
  "gene": "UniProtKB:P08134",
  "gene_symbol": "RHOC",
  "term_label": "cytosol"
}